CAP-Gly domain binding [GO:0071794] (molecular function) Sources: GOC:mah, InterPro:IPR000938 Relationships: is_a GO:0019904 Definition: Binding to a CAP-Gly domain of a protein. The CAP_Gly domain is a conserved, glycine-rich domain of about 42 residues found in some cytoskeleton-associated proteins, and features a novel protein fold containing three beta-sheets.